{
  "gene_symbol": "PI4KA",
  "term_id": "GO:0005886",
  "gene_name": "Phosphatidylinositol 4-kinase alpha",
  "gene": "UniProtKB:P42356",
  "term_label": "plasma membrane"
}